peptide metabolic process [GO:0006518] (biological process) Also known as: peptide metabolism Sources: GOC:go_curators Definition: The chemical reactions and pathways involving peptides, compounds of two or more amino acids where the alpha carboxyl group of one is bound to the alpha amino group of another. Subtypes: peptide modification [GO:0031179], GO:0043043, peptide catabolic process [GO:0043171], peptide stabilization [GO:0050822] Relationships: is a type of metabolic process [GO:0008152]